{
  "gene_name": "Electroneutral sodium bicarbonate exchanger 1",
  "gene": "UniProtKB:Q2Y0W8",
  "gene_symbol": "SLC4A8",
  "term_label": "sodium:bicarbonate symporter activity",
  "term_id": "GO:0008510"
}